{
  "gene_name": "RNA-binding region-containing protein 3",
  "gene": "UniProtKB:Q96LT9",
  "gene_symbol": "RNPC3",
  "term_label": "U12 snRNA binding",
  "term_id": "GO:0030626"
}